G protein-coupled adenosine receptor activity [GO:0001609] (molecular function) Relationships: is a type of GO:0004930; is part of GO:0001973 References: PMID:9755289 Sources: GOC:bf, GOC:mah Also known as: adenosine nucleotide receptor, G protein coupled adenosine receptor activity, G-protein coupled adenosine receptor activity, P1 receptor, adenosine receptor activity, G protein coupled, adenosine receptor activity, G-protein coupled, A1 adenosine receptor activity, G protein coupled, A1 adenosine receptor activity, G-protein coupled, A2A adenosine receptor activity, G protein coupled, A2A adenosine receptor activity, G-protein coupled, A2B adenosine receptor activity, G protein coupled, A2B adenosine receptor activity, G-protein coupled, A3 adenosine receptor activity, G protein coupled, A3 adenosine receptor activity, G-protein coupled, G protein coupled A1 adenosine receptor activity, G protein coupled A2A adenosine receptor activity, G protein coupled A2B adenosine receptor activity, G protein coupled A3 adenosine receptor activity, G-protein-coupled A1 adenosine receptor activity, G-protein-coupled A2A adenosine receptor activity, G-protein-coupled A2B adenosine receptor activity, G-protein-coupled A3 adenosine receptor activity Definition: Combining with adenosine and transmitting the signal across the membrane by activating an associated G-protein; promotes the exchange of GDP for GTP on the alpha subunit of a heterotrimeric G-protein complex.